{
  "term_label": "defense response to Gram-negative bacterium",
  "gene_symbol": "CST11",
  "gene_name": "Cystatin-11",
  "gene": "UniProtKB:Q9H112",
  "term_id": "GO:0050829"
}